{
  "term_id": "GO:0003924",
  "gene": "UniProtKB:O95837",
  "gene_symbol": "GNA14",
  "term_label": "GTPase activity",
  "gene_name": "Guanine nucleotide-binding protein subunit alpha-14"
}